regulation of hemicellulose catabolic process [GO:2000988] (biological process) Relationships: is a type of regulation of polysaccharide metabolic process [GO:0032881]; is a type of GO:0043470; RO_0002211 hemicellulose catabolic process [GO:2000895] Sources: GOC:mengo_curators Definition: Any process that modulates the frequency, rate or extent of hemicellulose catabolic process. Also known as: regulation of hemicellulose catabolism Subtypes: regulation of xyloglucan catabolic process [GO:2000951], negative regulation of hemicellulose catabolic process [GO:2000989], positive regulation of hemicellulose catabolic process [GO:2000990], regulation of xylan catabolic process [GO:2001000]